{
  "term_label": "Unknown molecular function",
  "gene_symbol": "LRRC37A2",
  "gene": "UniProtKB:A6NM11",
  "gene_name": "Leucine-rich repeat-containing protein 37A2",
  "term_id": "UNKNOWN:0001"
}